{
  "gene_name": "Annexin A8-like protein 1",
  "gene": "UniProtKB:Q5VT79",
  "term_label": "endosomal transport",
  "term_id": "GO:0016197",
  "gene_symbol": "ANXA8L1"
}